{
  "gene_name": "Plastin-1",
  "term_label": "actin filament",
  "gene": "UniProtKB:Q14651",
  "gene_symbol": "PLS1",
  "term_id": "GO:0005884"
}